{
  "gene": "UniProtKB:Q96RE9",
  "gene_name": "Zinc finger protein 300",
  "term_id": "GO:0006357",
  "term_label": "regulation of transcription by RNA polymerase II",
  "gene_symbol": "ZNF300"
}